{
  "gene": "UniProtKB:O15344",
  "gene_name": "E3 ubiquitin-protein ligase Midline-1",
  "gene_symbol": "MID1",
  "term_label": "cytoplasm",
  "term_id": "GO:0005737"
}